{
  "term_id": "GO:0005634",
  "gene_symbol": "PRKAA2",
  "gene_name": "5'-AMP-activated protein kinase catalytic subunit alpha-2",
  "gene": "UniProtKB:P54646",
  "term_label": "nucleus"
}